{
  "term_id": "GO:0035330",
  "gene_symbol": "NEK8",
  "gene_name": "Serine_threonine-protein kinase Nek8",
  "term_label": "regulation of hippo signaling",
  "gene": "UniProtKB:Q86SG6"
}